{
  "gene": "UniProtKB:Q99619",
  "term_id": "GO:0043161",
  "term_label": "proteasome-mediated ubiquitin-dependent protein catabolic process",
  "gene_name": "SPRY domain-containing SOCS box protein 2",
  "gene_symbol": "SPSB2"
}